nucleotide-sugar biosynthetic process [GO:0009226] (biological process) Sources: ISBN:0198506732 Subtypes: UDP-N-acetylglucosamine biosynthetic process [GO:0006048], CMP-N-acetylneuraminate biosynthetic process [GO:0006055], GO:0006065, GDP-mannose biosynthetic process [GO:0009298], UDP-rhamnose biosynthetic process [GO:0010253], GO:0019277, GO:0019305, GDP-D-rhamnose biosynthetic process [GO:0019306], dTDP-mannose biosynthetic process [GO:0019308], GO:0033320, GO:0033352, UDP-L-arabinose biosynthetic process [GO:0033358], CMP-keto-3-deoxy-D-manno-octulosonic acid biosynthetic process [GO:0033468], GDP-L-galactose biosynthetic process [GO:0033472], GO:0033480, GO:0042350, GO:0052574, ADP-L-glycero-beta-D-manno-heptose biosynthetic process [GO:0097171], UDP-alpha-D-glucose biosynthetic process [GO:0120530], UDP-4-deoxy-4-formamido-beta-L-arabinopyranose biosynthetic process [GO:2001315] Also known as: nucleotide-sugar anabolism, nucleotide-sugar biosynthesis, nucleotide-sugar formation, nucleotide-sugar synthesis Relationships: is a type of GO:0009225; is_a carbohydrate derivative biosynthetic process [GO:1901137]; is a type of GO:1901293 Definition: The chemical reactions and pathways resulting in the formation of nucleotide-sugars, any nucleotide-carbohydrate in which the distal phosphoric residue of a nucleoside 5'-diphosphate is in glycosidic linkage with a monosaccharide or monosaccharide derivative.